{
  "gene_name": "Angiopoietin-2",
  "gene_symbol": "ANGPT2",
  "gene": "UniProtKB:O15123",
  "term_id": "GO:0031012",
  "term_label": "extracellular matrix"
}